{
  "term_id": "GO:0010719",
  "gene_symbol": "USF3",
  "gene": "UniProtKB:Q68DE3",
  "term_label": "negative regulation of epithelial to mesenchymal transition",
  "gene_name": "Basic helix-loop-helix domain-containing protein USF3"
}